negative regulation of phosphatidylinositol biosynthetic process [GO:0010512] (biological process) Definition: Any process that decreases the frequency, rate or extent of the chemical reactions and pathways resulting in the formation of phosphatidylinositol. Sources: GOC:dph, GOC:tb, GOC:vw Relationships: is_a regulation of phosphatidylinositol biosynthetic process [GO:0010511]; is a type of negative regulation of phospholipid biosynthetic process [GO:0071072]; RO_0002212 phosphatidylinositol biosynthetic process [GO:0006661] Subtypes: negative regulation of 1-phosphatidyl-1D-myo-inositol 4,5-bisphosphate biosynthetic process [GO:1902647]